monocyte chemotactic protein-1 production [GO:0071605] (biological process) Relationships: is a type of chemokine production [GO:0032602] Sources: GOC:add, GOC:rv Also known as: CCL2 production, MCP-1 production Definition: The appearance of monocyte chemotactic protein-1 due to biosynthesis or secretion following a cellular stimulus, resulting in an increase in its intracellular or extracellular levels. Regulation: regulated by regulation of monocyte chemotactic protein-1 production [GO:0071637]; negatively regulated by negative regulation of monocyte chemotactic protein-1 production [GO:0071638]; positively regulated by GO:0071639